{
  "term_id": "GO:0005737",
  "gene": "UniProtKB:Q8IUG5",
  "term_label": "cytoplasm",
  "gene_symbol": "MYO18B",
  "gene_name": "Unconventional myosin-XVIIIb"
}